RNA cytidine-uridine insertion [GO:0070712] (biological process) Definition: The modification of an RNA molecule by insertion of an cytidine-uridine dinucleotide. Sources: GOC:cb, GOC:mah Also known as: RNA CU insertion Relationships: is a type of RNA dinucleotide insertion [GO:0070707]